{
  "term_label": "negative regulation of osteoclast differentiation",
  "term_id": "GO:0045671",
  "gene_symbol": "GPR137",
  "gene_name": "Integral membrane protein GPR137",
  "gene": "UniProtKB:Q96N19"
}